{
  "term_id": "GO:0048019",
  "gene_name": "Humanin-like 9",
  "gene_symbol": "MTRNR2L9",
  "term_label": "receptor antagonist activity",
  "gene": "UniProtKB:P0CJ76"
}